{
  "gene_symbol": "UBAP1L",
  "term_label": "ubiquitin-dependent protein catabolic process via the multivesicular body sorting pathway",
  "gene_name": "Ubiquitin-associated protein 1-like",
  "term_id": "GO:0043162",
  "gene": "UniProtKB:F5GYI3"
}